{
  "gene_name": "DmX-like protein 2",
  "term_id": "UNKNOWN:0001",
  "gene_symbol": "DMXL2",
  "term_label": "Unknown molecular function",
  "gene": "UniProtKB:Q8TDJ6"
}